{
  "gene_symbol": "ZNF761",
  "gene_name": "Zinc finger protein 761",
  "gene": "UniProtKB:Q86XN6",
  "term_id": "GO:0005634",
  "term_label": "nucleus"
}